{
  "gene": "UniProtKB:Q9GZZ1",
  "term_id": "GO:0031415",
  "gene_symbol": "NAA50",
  "gene_name": "N-alpha-acetyltransferase 50",
  "term_label": "NatA complex"
}